granzyme B production [GO:0071613] (biological process) Definition: The appearance of granzyme B due to biosynthesis or secretion following a cellular stimulus, resulting in an increase in its intracellular or extracellular levels. Note: Note that this term is in the subset of terms that should not be used for direct gene product annotation. Instead, select one of the 'regulation' children terms. Sources: GOC:add, GOC:rv Relationships: is a type of GO:0002440 Regulation: regulated by GO:0071661; negatively regulated by negative regulation of granzyme B production [GO:0071662]; positively regulated by positive regulation of granzyme B production [GO:0071663]